{
  "gene_name": "Metallothionein-4",
  "term_id": "GO:0071294",
  "term_label": "cellular response to zinc ion",
  "gene": "UniProtKB:P47944",
  "gene_symbol": "MT4"
}